{
  "gene": "UniProtKB:Q9UP95",
  "gene_name": "Solute carrier family 12 member 4",
  "term_id": "GO:1902476",
  "term_label": "chloride transmembrane transport",
  "gene_symbol": "SLC12A4"
}